{
  "term_id": "GO:0005634",
  "gene": "UniProtKB:Q9H816",
  "gene_name": "5' exonuclease Apollo",
  "gene_symbol": "DCLRE1B",
  "term_label": "nucleus"
}